regulation of cell proliferation in bone marrow [GO:0071863] (biological process) Also known as: regulation of bone marrow cell proliferation References: PMID:17063141 Sources: GOC:mah, GOC:yaf Subtypes: GO:0071864, negative regulation of cell proliferation in bone marrow [GO:1903769] Definition: A process that modulates the frequency, rate or extent of cell proliferation in the bone marrow. Relationships: is a type of regulation of cell population proliferation [GO:0042127]; regulates GO:0071838